{
  "term_label": "intestinal cholesterol absorption",
  "term_id": "GO:0030299",
  "gene_name": "NPC intracellular cholesterol transporter 1",
  "gene_symbol": "NPC1",
  "gene": "UniProtKB:O15118"
}